regulation of lymphocyte proliferation [GO:0050670] (biological process) Relationships: is a type of regulation of mononuclear cell proliferation [GO:0032944]; is a type of regulation of lymphocyte activation [GO:0051249]; regulates GO:0046651 Definition: Any process that modulates the frequency, rate or extent of lymphocyte proliferation. Subtypes: regulation of B cell proliferation [GO:0030888], regulation of natural killer cell proliferation [GO:0032817], regulation of T cell proliferation [GO:0042129], GO:0050671, negative regulation of lymphocyte proliferation [GO:0050672] Sources: GOC:ai